{
  "term_label": "cytosol",
  "gene_symbol": "PRKAR2B",
  "gene": "UniProtKB:P31323",
  "term_id": "GO:0005829",
  "gene_name": "cAMP-dependent protein kinase type II-beta regulatory subunit"
}